negative regulation of myeloid progenitor cell differentiation [GO:1905454] (biological process) References: PMID:27010503 Sources: GOC:TermGenie, GO_REF:0000058 Also known as: down regulation of myeloid progenitor cell differentiation, down-regulation of myeloid progenitor cell differentiation, downregulation of myeloid progenitor cell differentiation, inhibition of myeloid progenitor cell differentiation Relationships: is a type of negative regulation of hematopoietic progenitor cell differentiation [GO:1901533]; is a type of regulation of myeloid progenitor cell differentiation [GO:1905453]; negatively regulates GO:0002318 Definition: Any process that stops, prevents or reduces the frequency, rate or extent of myeloid progenitor cell differentiation.